phosphatidylglycerol-prolipoprotein diacylglyceryl transferase activity [GO:0008961] (MF) References: PMID:8051048 Sources: RHEA:56712 Definition: Catalysis of the transfer of the diacylglyceryl group from phosphatidylglycerol to the sulfhydryl group of the prospective N-terminal cysteine residue in an unmodified prolipoprotein. Relationships: is a type of GO:0016757; is a type of GO:0140096